{
  "gene": "UniProtKB:Q5GH76",
  "term_id": "GO:1902742",
  "term_label": "apoptotic process involved in development",
  "gene_symbol": "XKR4",
  "gene_name": "XK-related protein 4"
}